negative regulation of shade avoidance [GO:1902447] (BP) Relationships: is a type of GO:0048585; is a type of regulation of shade avoidance [GO:1902446]; negatively regulates shade avoidance [GO:0009641] References: PMID:23763263 Sources: GOC:TermGenie Also known as: down regulation of shade avoidance, down-regulation of shade avoidance, downregulation of shade avoidance, inhibition of shade avoidance Definition: Any process that stops, prevents or reduces the frequency, rate or extent of shade avoidance.